{
  "gene_symbol": "CDH6",
  "term_id": "GO:0008013",
  "gene": "UniProtKB:P55285",
  "gene_name": "Cadherin-6",
  "term_label": "beta-catenin binding"
}